GDP-mannose biosynthetic process [GO:0009298] (biological process) Relationships: is a type of nucleotide-sugar biosynthetic process [GO:0009226]; is_a GO:0019673; has part GO:0004615 Subtypes: GDP-mannose biosynthetic process from mannose [GO:0061728], GDP-D-mannose biosynthetic process from fructose-6-phosphate [GO:0061729] Sources: GOC:ai Definition: The chemical reactions and pathways resulting in the formation of GDP-mannose, a substance composed of mannose in glycosidic linkage with guanosine diphosphate. Also known as: GDP-mannose anabolism, GDP-mannose biosynthesis, GDP-mannose formation, GDP-mannose synthesis